{
  "term_id": "GO:0140597",
  "gene_name": "Ankyrin repeat domain-containing protein 13C",
  "gene": "UniProtKB:Q8N6S4",
  "term_label": "protein carrier chaperone",
  "gene_symbol": "ANKRD13C"
}